regulation of receptor binding [GO:1900120] (biological process) Also known as: regulation of receptor ligand Relationships: is_a regulation of protein binding [GO:0043393]; regulates signaling receptor binding [GO:0005102] Sources: GOC:TermGenie, GOC:signaling Subtypes: regulation of cytokine activity [GO:0060300], negative regulation of receptor binding [GO:1900121] Definition: Any process that modulates the frequency, rate or extent of a protein or other molecule binding to a receptor.